{
  "gene_symbol": "USO1",
  "term_label": "membrane fusion",
  "term_id": "GO:0061025",
  "gene_name": "General vesicular transport factor p115",
  "gene": "UniProtKB:O60763"
}